transepithelial water transport [GO:0035377] (BP) Relationships: is a type of water transport [GO:0006833]; is a type of epithelial fluid transport [GO:0042045] Definition: The directed movement of water (H2O) from one side of an epithelium to the other. Sources: GOC:yaf